{
  "gene_symbol": "NDUFB3",
  "gene_name": "NADH dehydrogenase [ubiquinone] 1 beta subcomplex subunit 3",
  "term_id": "GO:0045271",
  "gene": "UniProtKB:O43676",
  "term_label": "respiratory chain complex I"
}